{
  "gene": "UniProtKB:Q8NDW4",
  "gene_symbol": "ZNF248",
  "gene_name": "Zinc finger protein 248",
  "term_label": "nucleus",
  "term_id": "GO:0005634"
}